{
  "gene_name": "Liver carboxylesterase 1",
  "term_label": "retinyl-palmitate esterase activity",
  "term_id": "GO:0050253",
  "gene": "UniProtKB:P23141",
  "gene_symbol": "CES1"
}